{
  "term_id": "GO:0005737",
  "gene_name": "Serine_threonine-protein kinase ULK1",
  "gene": "UniProtKB:O75385",
  "term_label": "cytoplasm",
  "gene_symbol": "ULK1"
}